{
  "gene": "UniProtKB:O00584",
  "gene_name": "Ribonuclease T2",
  "gene_symbol": "RNASET2",
  "term_id": "GO:0004521",
  "term_label": "RNA endonuclease activity"
}